{
  "term_label": "regulation of neuron projection development",
  "gene_name": "Nuclear distribution protein nudE-like 1",
  "term_id": "GO:0010975",
  "gene": "UniProtKB:Q9GZM8",
  "gene_symbol": "NDEL1"
}